host cell mitochondrial intermembrane space [GO:0072492] (cellular component) Relationships: is a type of host cell cytoplasm part [GO:0033655]; is part of host cell mitochondrial envelope [GO:0044190] Definition: The region between the inner and outer lipid bilayers of the host cell mitochondrial envelope. Sources: GOC:ecd